{
  "gene": "UniProtKB:A0A087X1C5",
  "term_label": "arachidonate metabolic process",
  "gene_name": "Putative cytochrome P450 2D7",
  "gene_symbol": "CYP2D7",
  "term_id": "GO:0019369"
}